nitrogenase complex [GO:0016610] (cellular component) Definition: An enzyme complex composed of two proteins, dinitrogenase and nitrogenase reductase; dinitrogenase is tetrameric with an alpha2-beta2 structure and nitrogenase reductase is a homodimer, and both are associated with metal ions, which differ between species. Both proteins are required for the enzyme activity of the complex, the formation of oxidized ferredoxin and ammonia from reduced ferredoxin and nitrogen. Relationships: is a type of intracellular protein-containing complex [GO:0140535]; is a type of oxidoreductase complex [GO:1990204] References: PMID:10852721 Subtypes: iron-iron nitrogenase complex [GO:0016611], molybdenum-iron nitrogenase complex [GO:0016612], GO:0016613